mitochondrial calcium ion homeostasis [GO:0051560] (BP) Also known as: calcium ion homeostasis in mitochondria, calcium ion homeostasis in mitochondrion, mitochondrial calcium ion concentration regulation, regulation of calcium ion concentration in mitochondria, regulation of calcium ion concentration in mitochondrion, regulation of mitochondrial calcium ion concentration Sources: GOC:ai, GOC:mah Relationships: is a type of intracellular calcium ion homeostasis [GO:0006874]; BFO_0000066 GO:0005739 Subtypes: positive regulation of mitochondrial calcium ion concentration [GO:0051561], negative regulation of mitochondrial calcium ion concentration [GO:0051562] Definition: Any process involved in the maintenance of an internal steady state of calcium ions within the cytoplasm of a cell or between mitochondria and their surroundings.